nociceptin receptor activity [GO:0001626] (molecular function) Relationships: is a type of G protein-coupled opioid receptor activity [GO:0004985]; is a type of G protein-coupled peptide receptor activity [GO:0008528] Also known as: OFQ receptor activity, ORPH receptor, nociceptin/orphanin-FQ receptor activity, orphanin-FQ receptor activity, X-opioid receptor activity References: PMID:18670432 Sources: GOC:bf, GOC:mah Definition: Combining with the peptide nociceptin, and transmitting the signal across the membrane by activating an associated G-protein.